regulation of cellular localization [GO:0060341] (biological process) Definition: Any process that modulates the frequency, rate or extent of a process in which a cell, a substance, or a cellular entity is transported to, or maintained in a specific location within or in the membrane of a cell. Sources: GOC:dph, GOC:tb Also known as: regulation of cellular localisation Relationships: is a type of regulation of localization [GO:0032879]; is a type of GO:0050794; regulates GO:0051641 Subtypes: regulation of calcium ion transport into cytosol [GO:0010522], GO:0032386, regulation of vesicle targeting, to, from or within Golgi [GO:0048209], regulation of actin cortical patch localization [GO:0060583], regulation of insulin secretion involved in cellular response to glucose stimulus [GO:0061178], GO:0090313, GO:0150054, regulation of protein insertion into mitochondrial outer membrane [GO:1903636], regulation of plasma membrane raft polarization [GO:1903906], regulation of iron ion import across plasma membrane [GO:1904438], regulation of protein localization to membrane [GO:1905475], regulation of ribonucleoprotein complex localization [GO:2000197]